oxidoreductase activity, acting on paired donors, with incorporation or reduction of molecular oxygen, another compound as one donor, and incorporation of one atom of oxygen [GO:0016716] (molecular function) Definition: Catalysis of an oxidation-reduction (redox) reaction in which hydrogen or electrons are transferred from each of two donors, and one atom of oxygen is incorporated into one donor. Sources: EC:1.14.18.- Relationships: is a type of monooxygenase activity [GO:0004497]; is a type of GO:0016705 Subtypes: C-4 methylsterol oxidase activity [GO:0000254], tyrosinase activity [GO:0004503], CMP-N-acetylneuraminate monooxygenase activity [GO:0030338], cholesterol 26-hydroxylase activity [GO:0031073], GO:0050183, fatty acid 2-hydroxylase activity [GO:0080132], GO:0102772